{
  "gene": "UniProtKB:Q86Y07",
  "gene_name": "Serine_threonine-protein kinase VRK2",
  "term_label": "protein serine/threonine kinase activity",
  "gene_symbol": "VRK2",
  "term_id": "GO:0004674"
}